{
  "term_id": "GO:0030301",
  "gene_name": "StAR-related lipid transfer protein 3",
  "gene": "UniProtKB:Q14849",
  "gene_symbol": "STARD3",
  "term_label": "cholesterol transport"
}